positive regulation of formin-nucleated actin cable assembly [GO:0090338] (biological process) References: PMID:12810699, PMID:15923184 Sources: GOC:jh, GOC:tb Relationships: is a type of positive regulation of actin filament bundle assembly [GO:0032233]; is a type of regulation of formin-nucleated actin cable assembly [GO:0090337]; positively regulates formin-nucleated actin cable assembly [GO:0070649] Definition: Any process that increases the rate, frequency, or extent of formin-nucleated actin cable assembly. Formin-nucleated actin cable assembly is the aggregation, arrangement and bonding together of a set of components to form a formin-nucleated actin cable. A formin-nucleated actin cable is an actin filament bundle that consists of short filaments organized into bundles of uniform polarity, and is nucleated by formins.